{
  "term_id": "UNKNOWN:0001",
  "gene_name": "Putative uncharacterized protein LOC100128429",
  "gene_symbol": "Q6ZWC4",
  "gene": "UniProtKB:Q6ZWC4",
  "term_label": "Unknown molecular function"
}